male meiosis chromosome separation [GO:0051308] (biological process) Definition: The process in which paired chromosomes are physically detached from each other during male meiosis. Sources: GOC:ai Relationships: is_a male meiosis chromosome segregation [GO:0007060]; is a type of meiotic chromosome separation [GO:0051307] Also known as: chromosome separation during male meiosis, male meiosis chromosome resolution